{
  "gene": "UniProtKB:Q9C0C9",
  "term_label": "Unknown cellular component",
  "term_id": "UNKNOWN:0003",
  "gene_name": "(E3-independent) E2 ubiquitin-conjugating enzyme",
  "gene_symbol": "UBE2O"
}